meiotic strand displacement [GO:0000714] (biological process) References: PMID:10357855 Sources: GOC:elh Definition: The cell cycle process in which the broken 3' single-strand DNA molecule that formed heteroduplex DNA with its complement in an intact duplex DNA is rejected. The Watson-Crick base pairing in the original duplex is restored. The rejected 3' single-strand DNA molecule reanneals with its original complement to reform two intact duplex molecules. This occurs during meiosis. Also known as: meiotic D-loop dissociation, meiotic D-loop processing, meiotic displacement loop dissociation, meiotic displacement loop processing Relationships: is a type of GO:0000732; is a type of meiosis I cell cycle process [GO:0061982] Subtypes: meiotic strand displacement involved in double-strand break repair via SDSA [GO:1902346]